{
  "term_id": "GO:0005829",
  "gene_name": "Formin-like protein 3",
  "gene_symbol": "FMNL3",
  "gene": "UniProtKB:Q8IVF7",
  "term_label": "cytosol"
}